{
  "gene_symbol": "SLC12A2",
  "gene_name": "Solute carrier family 12 member 2",
  "gene": "UniProtKB:P55011",
  "term_label": "chloride ion homeostasis",
  "term_id": "GO:0055064"
}